{
  "term_id": "GO:0035025",
  "term_label": "positive regulation of Rho protein signal transduction",
  "gene_name": "Reticulon-4 receptor",
  "gene_symbol": "RTN4R",
  "gene": "UniProtKB:Q9BZR6"
}